muscle system process [GO:0003012] (BP) Regulation: regulated by regulation of muscle system process [GO:0090257] Also known as: muscle physiological process Definition: An organ system process carried out at the level of a muscle. Muscle tissue is composed of contractile cells or fibers. Relationships: is a type of GO:0003008 Sources: GOC:mtg_cardio Subtypes: muscle contraction [GO:0006936], muscle hypertrophy [GO:0014896], muscle adaptation [GO:0043500], relaxation of muscle [GO:0090075]